regulation of cardiac ventricle formation [GO:1904942] (biological process) Definition: Any process that modulates the frequency, rate or extent of cardiac ventricle formation. Subtypes: GO:1904943, positive regulation of cardiac ventricle formation [GO:1904944] References: PMID:23575307 Sources: GOC:BHF, GOC:BHF_miRNA, GOC:TermGenie, GOC:bc, GO_REF:0000058 Relationships: is a type of regulation of cardiac chamber formation [GO:1901210]; RO_0002211 cardiac ventricle formation [GO:0003211]